{
  "gene_symbol": "SARNP",
  "gene": "UniProtKB:P82979",
  "term_id": "GO:0016973",
  "gene_name": "SAP domain-containing ribonucleoprotein",
  "term_label": "poly(A)+ mRNA export from nucleus"
}